{
  "gene": "UniProtKB:P43681",
  "term_id": "GO:0007274",
  "gene_name": "Neuronal acetylcholine receptor subunit alpha-4",
  "gene_symbol": "CHRNA4",
  "term_label": "neuromuscular synaptic transmission"
}